vasoconstriction of artery involved in baroreceptor response to lowering of systemic arterial blood pressure [GO:0001987] (BP) Definition: A process that is triggered by vasomotor excitation and results in a decrease in the diameter of an artery during the baroreceptor response to decreased blood pressure. Sources: ISBN:0721643949 Relationships: is a type of vasoconstriction [GO:0042310]; is part of baroreceptor response to decreased systemic arterial blood pressure [GO:0001982]